{
  "gene": "UniProtKB:P05177",
  "term_id": "GO:0009404",
  "term_label": "toxin metabolic process",
  "gene_symbol": "CYP1A2",
  "gene_name": "Cytochrome P450 1A2"
}